{
  "gene_name": "Transcription elongation factor A protein 2",
  "gene_symbol": "TCEA2",
  "gene": "UniProtKB:Q15560",
  "term_label": "nucleus",
  "term_id": "GO:0005634"
}